{
  "gene": "UniProtKB:Q6IEV9",
  "gene_name": "Olfactory receptor 4C11",
  "term_id": "GO:0004984",
  "term_label": "olfactory receptor activity",
  "gene_symbol": "OR4C11"
}